{
  "gene": "UniProtKB:Q9Y6K5",
  "gene_symbol": "OAS3",
  "term_label": "membrane",
  "term_id": "GO:0016020",
  "gene_name": "2'-5'-oligoadenylate synthase 3"
}